{
  "term_label": "cytoplasmic vesicle membrane",
  "term_id": "GO:0030659",
  "gene_symbol": "TRARG1",
  "gene": "UniProtKB:Q8IXB3",
  "gene_name": "Trafficking regulator of GLUT4 1"
}